{
  "gene": "UniProtKB:P78559",
  "gene_name": "Microtubule-associated protein 1A",
  "term_label": "dendrite",
  "term_id": "GO:0030425",
  "gene_symbol": "MAP1A"
}